{
  "term_label": "positive regulation of calcium ion-dependent exocytosis",
  "gene_name": "Rab effector Noc2",
  "gene_symbol": "RPH3AL",
  "gene": "UniProtKB:Q9UNE2",
  "term_id": "GO:0045956"
}